{
  "gene_symbol": "DHRS4L1",
  "gene": "UniProtKB:P0CG22",
  "term_label": "peroxisome",
  "term_id": "GO:0005777",
  "gene_name": "Putative dehydrogenase_reductase SDR family member 4-like 1"
}